{
  "term_label": "dendrite self-avoidance",
  "term_id": "GO:0070593",
  "gene_name": "Neuroplastin",
  "gene_symbol": "NPTN",
  "gene": "UniProtKB:Q9Y639"
}